{
  "term_label": "plasma membrane",
  "gene": "UniProtKB:P41273",
  "gene_name": "Tumor necrosis factor ligand superfamily member 9",
  "term_id": "GO:0005886",
  "gene_symbol": "TNFSF9"
}